{
  "term_id": "UNKNOWN:0002",
  "gene_symbol": "TBC1D19",
  "gene": "UniProtKB:Q8N5T2",
  "gene_name": "TBC1 domain family member 19",
  "term_label": "Unknown biological process"
}